{
  "term_label": "Unknown cellular component",
  "gene": "UniProtKB:Q86TY3",
  "gene_symbol": "ARMH4",
  "term_id": "UNKNOWN:0003",
  "gene_name": "Armadillo-like helical domain-containing protein 4"
}